uropod membrane [GO:0031259] (cellular component) Relationships: is a type of cell projection membrane [GO:0031253]; is_a GO:0031257; BFO_0000050 uropod [GO:0001931] Also known as: uropodium membrane Sources: GOC:mah Definition: The portion of the plasma membrane surrounding a uropod.